{
  "gene": "UniProtKB:Q6UXY1",
  "gene_name": "Brain-specific angiogenesis inhibitor 1-associated protein 2-like protein 2",
  "term_label": "actin crosslink formation",
  "gene_symbol": "BAIAP2L2",
  "term_id": "GO:0051764"
}